{
  "term_label": "chromosome",
  "term_id": "GO:0005694",
  "gene_name": "RAD9, HUS1, RAD1-interacting nuclear orphan protein 1",
  "gene_symbol": "RHNO1",
  "gene": "UniProtKB:Q9BSD3"
}